{
  "gene": "UniProtKB:Q9UG01",
  "gene_name": "Intraflagellar transport protein 172 homolog",
  "gene_symbol": "IFT172",
  "term_label": "intraciliary transport particle B",
  "term_id": "GO:0030992"
}